{
  "gene_symbol": "GBP3",
  "gene_name": "Guanylate-binding protein 3",
  "term_id": "GO:0031410",
  "gene": "UniProtKB:Q9H0R5",
  "term_label": "cytoplasmic vesicle"
}